{
  "term_id": "GO:0005964",
  "gene_name": "Phosphorylase b kinase gamma catalytic chain, skeletal muscle_heart isoform",
  "term_label": "phosphorylase kinase complex",
  "gene": "UniProtKB:Q16816",
  "gene_symbol": "PHKG1"
}